{
  "term_id": "UNKNOWN:0003",
  "term_label": "Unknown cellular component",
  "gene_symbol": "NAT2",
  "gene": "UniProtKB:P11245",
  "gene_name": "Arylamine N-acetyltransferase 2"
}